interleukin-9 receptor activity [GO:0004919] (molecular function) Definition: Combining with interleukin-9 and transmitting the signal from one side of the membrane to the other to initiate a change in cell activity. Sources: GOC:jl, GOC:signaling Also known as: IL-9 receptor activity, IL-9R Relationships: is a type of cytokine receptor activity [GO:0004896]; is part of GO:0038113; BFO_0000051 interleukin-9 binding [GO:0019983]